FACIT collagen complex [GO:0140153] (cellular component) References: PMID:1882421, PMID:21421911 Relationships: is_a complex of collagen trimers [GO:0098644]; is part of collagenous component of interstitial matrix [GO:0140152] Definition: A supramolecular complex formed by fibril-associated collagens with interrupted triple helices (FACIT) that associate with collagen fibrils and forms a link on large, banded fibrils.